{
  "gene_name": "Tyrosine-protein kinase Tec",
  "gene_symbol": "TEC",
  "gene": "UniProtKB:P42680",
  "term_label": "plasma membrane",
  "term_id": "GO:0005886"
}